{
  "term_id": "GO:0003730",
  "gene_name": "Far upstream element-binding protein 2",
  "term_label": "mRNA 3'-UTR binding",
  "gene": "UniProtKB:Q92945",
  "gene_symbol": "KHSRP"
}